{
  "gene": "UniProtKB:Q86Y28",
  "gene_name": "B melanoma antigen 4",
  "gene_symbol": "BAGE4",
  "term_label": "Unknown molecular function",
  "term_id": "UNKNOWN:0001"
}